positive regulation of protein glutathionylation [GO:0010733] (biological process) Also known as: positive regulation of protein amino acid glutathionylation Relationships: is a type of regulation of protein glutathionylation [GO:0010732]; is_a positive regulation of protein modification process [GO:0031401]; positively regulates protein glutathionylation [GO:0010731] Definition: Any process that increases the rate, frequency, or extent of protein glutathionylation. Protein glutathionylation is the protein modification process in which a glutathione molecule is added to a protein amino acid through a disulfide linkage. Sources: GOC:BHF, GOC:dph, GOC:rl, GOC:tb